{
  "term_label": "protein targeting to membrane",
  "gene_name": "Rab proteins geranylgeranyltransferase component A 2",
  "gene_symbol": "CHML",
  "term_id": "GO:0006612",
  "gene": "UniProtKB:P26374"
}